{
  "gene_name": "C-X-C motif chemokine 3",
  "term_label": "Unknown cellular component",
  "gene_symbol": "CXCL3",
  "term_id": "UNKNOWN:0003",
  "gene": "UniProtKB:P19876"
}